{
  "term_label": "GTP binding",
  "term_id": "GO:0005525",
  "gene_name": "ADP-ribosylation factor-like protein 6",
  "gene": "UniProtKB:Q9H0F7",
  "gene_symbol": "ARL6"
}